{
  "gene_name": "Zinc finger protein 750",
  "term_label": "positive regulation of transcription by RNA polymerase II",
  "term_id": "GO:0045944",
  "gene_symbol": "ZNF750",
  "gene": "UniProtKB:Q32MQ0"
}